mRNA cleavage stimulating factor complex [GO:0005848] (cellular component) Definition: A protein complex required for mRNA cleavage but not for poly(A) addition. References: PMID:10357856 Sources: GOC:mah Also known as: CstF complex, cleavage stimulation factor activity Relationships: is a type of mRNA cleavage factor complex [GO:0005849]